regulation of iron ion transport [GO:0034756] (biological process) Relationships: is a type of regulation of metal ion transport [GO:0010959]; regulates iron ion transport [GO:0006826] Definition: Any process that modulates the frequency, rate or extent of the directed movement of iron ions (Fe) into, out of or within a cell, or between cells, by means of some agent such as a transporter or pore. Sources: GOC:mah Also known as: regulation of Fe transport, regulation of iron transport, regulation of iron import, regulation of iron ion import Subtypes: negative regulation of iron ion transport [GO:0034757], positive regulation of iron ion transport [GO:0034758], regulation of iron ion transmembrane transport [GO:0034759]